{
  "gene_symbol": "TET1",
  "gene_name": "Methylcytosine dioxygenase TET1",
  "term_id": "GO:0005634",
  "term_label": "nucleus",
  "gene": "UniProtKB:Q8NFU7"
}